{
  "term_id": "UNKNOWN:0002",
  "gene_symbol": "NBPF19",
  "gene_name": "Neuroblastoma breakpoint family member 19",
  "term_label": "Unknown biological process",
  "gene": "UniProtKB:A0A087WUL8"
}